regulation of convergent extension involved in notochord morphogenesis [GO:1904136] (biological process) Definition: Any process that modulates the frequency, rate or extent of convergent extension involved in notochord morphogenesis. Relationships: is a type of GO:1904103; regulates convergent extension involved in notochord morphogenesis [GO:1904126] Subtypes: negative regulation of convergent extension involved in notochord morphogenesis [GO:1904137], positive regulation of convergent extension involved in notochord morphogenesis [GO:1904138] References: PMID:24892953 Sources: GOC:TermGenie, GOC:dph, GO_REF:0000058